{
  "term_id": "GO:0030334",
  "term_label": "regulation of cell migration",
  "gene_name": "Fibroblast growth factor 21",
  "gene_symbol": "FGF21",
  "gene": "UniProtKB:Q9NSA1"
}